inner stripe development [GO:0072057] (biological process) Relationships: is a type of anatomical structure development [GO:0048856]; is part of GO:0072054 Definition: The process whose specific outcome is the progression of the inner stripe over time, from its formation to the mature structure. The inner stripe is a deep, centrally located portion of the renal outer medulla and is traversed by thin descending and thick ascending portions of the loops of Henle. Sources: GOC:mtg_kidney_jan10